{
  "gene": "UniProtKB:P52738",
  "gene_symbol": "ZNF140",
  "gene_name": "Zinc finger protein 140",
  "term_label": "regulation of transcription by RNA polymerase II",
  "term_id": "GO:0006357"
}